{
  "gene_symbol": "TAL2",
  "gene_name": "T-cell acute lymphocytic leukemia protein 2",
  "term_id": "UNKNOWN:0003",
  "term_label": "Unknown cellular component",
  "gene": "UniProtKB:Q16559"
}